{
  "gene_name": "Casein kinase I isoform epsilon",
  "gene": "UniProtKB:P49674",
  "term_id": "GO:0032436",
  "term_label": "positive regulation of proteasomal ubiquitin-dependent protein catabolic process",
  "gene_symbol": "CSNK1E"
}